{
  "term_label": "regulation of angiogenesis",
  "gene_name": "Tubulinyl-Tyr carboxypeptidase 1",
  "gene": "UniProtKB:Q7L8A9",
  "gene_symbol": "VASH1",
  "term_id": "GO:0045765"
}